{
  "gene_name": "Kinesin-like protein KIF28P",
  "term_id": "GO:0003777",
  "gene_symbol": "KIF28P",
  "term_label": "microtubule motor activity",
  "gene": "UniProtKB:B7ZC32"
}